{
  "term_label": "Unknown molecular function",
  "term_id": "UNKNOWN:0001",
  "gene": "UniProtKB:Q8NA23",
  "gene_symbol": "WDR31",
  "gene_name": "WD repeat-containing protein 31"
}